{
  "gene_symbol": "IRS2",
  "term_label": "cytosol",
  "term_id": "GO:0005829",
  "gene": "UniProtKB:Q9Y4H2",
  "gene_name": "Insulin receptor substrate 2"
}